adiponectin binding [GO:0055100] (molecular function) Relationships: is a type of GO:0005515; is a type of hormone binding [GO:0042562] References: PMID:15210937 Sources: GOC:BHF, GOC:rl Definition: Binding to adiponectin, a protein hormone produced by adipose tissue that modulates a number of metabolic processes, including glucose regulation and fatty acid catabolism.